{
  "gene_name": "Zinc finger protein 646",
  "term_label": "Unknown cellular component",
  "gene_symbol": "ZNF646",
  "term_id": "UNKNOWN:0003",
  "gene": "UniProtKB:O15015"
}